inositol 3-kinase activity [GO:0019140] (molecular function) Also known as: myoinositol kinase activity, myo-inositol 3-kinase activity, ATP:myo-inositol 1-phosphotransferase activity, inositol 1-kinase activity, inositol-1-kinase (phosphorylating), myo-inositol 1-kinase activity Relationships: is_a kinase activity [GO:0016301]; is a type of phosphotransferase activity, alcohol group as acceptor [GO:0016773] Definition: Catalysis of the reaction: ATP + myo-inositol = ADP + 1D-myo-inositol 3-phosphate. Sources: EC:2.7.1.64